{
  "term_id": "UNKNOWN:0001",
  "gene_name": "Coiled-coil domain-containing protein 82",
  "gene_symbol": "CCDC82",
  "gene": "UniProtKB:Q8N4S0",
  "term_label": "Unknown molecular function"
}